AMP metabolic process [GO:0046033] (biological process) Definition: The chemical reactions and pathways involving AMP, adenosine monophosphate. Sources: GOC:go_curators Also known as: AMP metabolism, adenylate forming enzyme activity Relationships: is a type of purine ribonucleotide metabolic process [GO:0009150]; is a type of purine ribonucleoside monophosphate metabolic process [GO:0009167] Subtypes: GO:0006167, AMP catabolic process [GO:0006196], GO:0006756